{
  "gene_name": "LIX1-like protein",
  "gene": "UniProtKB:Q8IVB5",
  "term_id": "GO:0097352",
  "gene_symbol": "LIX1L",
  "term_label": "autophagosome maturation"
}